{
  "gene_name": "Amyloid-beta A4 precursor protein-binding family B member 3",
  "term_label": "regulation of DNA-templated transcription",
  "term_id": "GO:0006355",
  "gene_symbol": "APBB3",
  "gene": "UniProtKB:O95704"
}